{
  "term_id": "UNKNOWN:0001",
  "term_label": "Unknown molecular function",
  "gene_name": "LRRN4 C-terminal-like protein",
  "gene": "UniProtKB:Q8ND94",
  "gene_symbol": "LRRN4CL"
}